{
  "gene": "UniProtKB:P62330",
  "gene_symbol": "ARF6",
  "gene_name": "ADP-ribosylation factor 6",
  "term_id": "GO:0060998",
  "term_label": "regulation of dendritic spine development"
}